{
  "gene_name": "Cell division control protein 42 homolog",
  "term_id": "GO:0003924",
  "gene_symbol": "CDC42",
  "gene": "UniProtKB:P60953",
  "term_label": "GTPase activity"
}